{
  "gene_name": "Centrosomal protein of 290 kDa",
  "gene_symbol": "CEP290",
  "term_id": "UNKNOWN:0001",
  "term_label": "Unknown molecular function",
  "gene": "UniProtKB:O15078"
}